{
  "gene": "UniProtKB:P46379",
  "term_id": "GO:0036503",
  "term_label": "ERAD pathway",
  "gene_name": "Large proline-rich protein BAG6",
  "gene_symbol": "BAG6"
}